regulation of tube size [GO:0035150] (biological process) Relationships: is a type of regulation of anatomical structure size [GO:0090066] Subtypes: GO:0035151, regulation of tube diameter [GO:0035296], regulation of Malpighian tubule size [GO:0035298] References: PMID:10887083 Definition: Ensuring that a tube is of the correct length and diameter. Tube size must be maintained not only during tube formation, but also throughout development and in some physiological processes.